{
  "term_id": "GO:0032497",
  "gene_name": "Lymphocyte antigen 96",
  "gene": "UniProtKB:Q9Y6Y9",
  "term_label": "detection of lipopolysaccharide",
  "gene_symbol": "LY96"
}